tRNA 5-taurinomethyluridine synthase activity [GO:0160236] (molecular function) Definition: Catalysis of the reaction: 5,10-methylenetetrahydrofolate + taurine + GTP + H2O + uridine34 in tRNA + A = 7,8-dihydrofolate + GDP + phosphate + 5-taurinomethyluridine34 in tRNA + H+ + AH2. References: PMID:29390138, PMID:33619562 Sources: RHEA:83279 Relationships: is a type of transferase activity [GO:0016740]; is a type of catalytic activity, acting on a tRNA [GO:0140101]